lysosome fission [GO:0170064] (biological process) References: PMID:31171420, PMID:38538795 Definition: The process by which lysosomes undergo budding and fission to maintain their steady-state number, shape, size, composition and function, and to accomplish regeneration. Relationships: is a type of organelle fission [GO:0048285]